negative regulation of phosphatidylinositol-3,4,5-trisphosphate 5-phosphatase activity [GO:2001145] (biological process) Relationships: is a type of GO:0010923; negatively regulates phosphatidylinositol-3,4,5-trisphosphate 5-phosphatase activity [GO:0034485] Definition: Any process that stops, prevents or reduces the frequency, rate or extent of phosphatidylinositol-3,4,5-trisphosphate 5-phosphatase activity. Sources: GOC:obol